positive regulation of spore germination [GO:1904361] (biological process) Relationships: is a type of GO:0048522; is a type of positive regulation of developmental process [GO:0051094]; is a type of regulation of spore germination [GO:1904359]; positively regulates spore germination [GO:0009847] Subtypes: GO:0075228 References: PMID:14718564, PMID:8798577 Sources: GOC:TermGenie, GO_REF:0000058 Definition: Any process that activates or increases the frequency, rate or extent of spore germination. Also known as: up regulation of spore germination, up-regulation of spore germination, upregulation of spore germination, activation of spore germination, positive regulation of spore germination on or near host